(R)-2-hydroxyisocaproate dehydrogenase activity [GO:0043713] (molecular function) Definition: Catalysis of the reaction: 2-oxoisocaproate + NADH + H+ = (R)-2-hydroxyisocaproate + NAD+. Relationships: is a type of oxidoreductase activity, acting on the CH-OH group of donors, NAD or NADP as acceptor [GO:0016616] References: PMID:16957230 Sources: GOC:jl